CDP-2,3-bis-(O-geranylgeranyl)-sn-glycerol synthase activity [GO:0043338] (molecular function) Also known as: CDP-2,3-di-O-geranylgeranyl-sn-glycerol synthase, CTP:2,3-di-O-geranylgeranyl-sn-glycero-1-phosphate cytidyltransferase activity Definition: Catalysis of the reaction: 2,3-bis-O-(geranylgeranyl)-sn-glycerol 1-phosphate + CTP + H+ = CDP-2,3-bis-O-(geranylgeranyl)-sn-glycerol + diphosphate. References: PMID:10960477 Sources: GOC:jl, RHEA:25690 Relationships: is a type of GO:0070567